fatty alcohol metabolic process [GO:1903173] (biological process) Subtypes: GO:0006070, phytol metabolic process [GO:0033306], GO:1903174, fatty alcohol biosynthetic process [GO:1903175] References: PMID:24036493 Sources: GOC:TermGenie, GOC:mengo_curators, GO_REF:0000068 Relationships: is a type of alcohol metabolic process [GO:0006066]; is a type of fatty acid derivative metabolic process [GO:1901568] Also known as: fatty alcohol metabolism Definition: The chemical reactions and pathways involving fatty alcohol.